isopentenyl-diphosphate delta-isomerase activity [GO:0004452] (molecular function) Definition: Catalysis of the reaction: isopentenyl diphosphate = dimethylallyl diphosphate. Sources: RHEA:23284 Also known as: isopentenyl-diphosphate D-isomerase activity, IPP isomerase activity, isopentenyl-diphosphate delta3-delta2-isomerase activity, isopentenylpyrophosphate delta-isomerase activity, isopentenylpyrophosphate isomerase activity, methylbutenylpyrophosphate isomerase activity Relationships: is a type of intramolecular oxidoreductase activity, transposing C=C bonds [GO:0016863]